positive regulation of hydrogen peroxide biosynthetic process [GO:0010729] (biological process) Definition: Any process that increases the rate, frequency or extent of hydrogen peroxide biosynthesis. The chemical reactions and pathways resulting in the formation of hydrogen peroxide (H2O2), a potentially harmful byproduct of aerobic cellular respiration which can cause damage to DNA. Sources: GOC:dph, GOC:hjd, GOC:tb Also known as: positive regulation of hydrogen peroxide biosynthesis Relationships: is a type of regulation of hydrogen peroxide biosynthetic process [GO:0010728]; is a type of positive regulation of reactive oxygen species biosynthetic process [GO:1903428]; positively regulates hydrogen peroxide biosynthetic process [GO:0050665]